{
  "gene_name": "UBX domain-containing protein 6",
  "gene": "UniProtKB:Q9BZV1",
  "gene_symbol": "UBXN6",
  "term_label": "Unknown biological process",
  "term_id": "UNKNOWN:0002"
}